{
  "term_id": "GO:0015711",
  "gene": "UniProtKB:Q9NSA0",
  "gene_symbol": "SLC22A11",
  "term_label": "organic anion transport",
  "gene_name": "Solute carrier family 22 member 11"
}